UDP-N-acetylmuramate-L-alanyl-gamma-D-glutamyl-meso-2,6-diaminoheptanedioate ligase activity [GO:0106418] (molecular function) References: PMID:17384195, PMID:8808921 Sources: RHEA:29563 Definition: Catalysis of the reaction: ATP + UDP-N-acetyl-alpha-D-muramate + L-alanyl-gamma-D-glutamyl-meso-2,6-diaminoheptanedioate = ADP + phosphate + UDP-N-acetylmuramoyl-L-alanyl-gamma-D-glutamyl-meso-2,6-diaminoheptanedioate. Relationships: is a type of acid-amino acid ligase activity [GO:0016881] Also known as: murein peptide ligase